isopenicillin-N synthase activity [GO:0016216] (molecular function) Relationships: is a type of GO:0046993 Definition: Catalysis of the reaction: N-[(5S)-5-amino-5-carboxypentanoyl]-L-cysteinyl-D-valine + O2 = 2 H2O + isopenicillin N. Sources: EC:1.21.3.1, RHEA:22428 Also known as: isopenicillin-N synthetase activity, N-[(5S)-5-amino-5-carboxypentanoyl]-L-cysteinyl-D-valine:oxygen oxidoreductase (cyclizing), isopenicillin N synthase activity